leucoplast [GO:0009516] (cellular component) Subtypes: GO:0009545, proteinoplast [GO:0031986] Sources: ISBN:0943088399 Definition: A colorless plastid involved in the synthesis of monoterpenes. Relationships: is a type of plastid [GO:0009536]